{
  "term_label": "serine-type endopeptidase activity",
  "gene": "UniProtKB:O43240",
  "term_id": "GO:0004252",
  "gene_name": "Kallikrein-10",
  "gene_symbol": "KLK10"
}